{
  "gene_name": "Guided entry of tail-anchored proteins factor CAMLG",
  "gene_symbol": "CAMLG",
  "term_label": "Unknown molecular function",
  "term_id": "UNKNOWN:0001",
  "gene": "UniProtKB:P49069"
}